chemoattractant activity [GO:0042056] (molecular function) Subtypes: chemoattractant activity involved in axon guidance [GO:1902379] Definition: Providing the environmental signal that initiates the directed movement of a motile cell or organism towards a higher concentration of that signal. Sources: GOC:go_curators, ISBN:0198506732 Also known as: attractant Relationships: is a type of receptor ligand activity [GO:0048018]; is part of positive chemotaxis [GO:0050918]